{
  "gene_symbol": "TMEM65",
  "gene": "UniProtKB:Q6PI78",
  "gene_name": "Transmembrane protein 65",
  "term_label": "Unknown molecular function",
  "term_id": "UNKNOWN:0001"
}